{
  "gene": "UniProtKB:Q6YN16",
  "term_id": "UNKNOWN:0002",
  "gene_symbol": "HSDL2",
  "term_label": "Unknown biological process",
  "gene_name": "Hydroxysteroid dehydrogenase-like protein 2"
}